regulation of wound healing [GO:0061041] (biological process) Relationships: is a type of regulation of response to wounding [GO:1903034]; regulates GO:0042060 Definition: Any process that modulates the rate, frequency, or extent of the series of events that restore integrity to a damaged tissue, following an injury. Sources: GOC:BHF, GOC:dph Subtypes: regulation of blood coagulation [GO:0030193], regulation of vascular wound healing [GO:0061043], negative regulation of wound healing [GO:0061045], positive regulation of wound healing [GO:0090303], regulation of wound healing, spreading of epidermal cells [GO:1903689]